structural constituent of egg coat [GO:0035804] (molecular function) References: PMID:16944418, PMID:17163408 Definition: The action of a molecule that contributes to the structural integrity of an egg coat. An egg coat is a specialized extracellular matrix that surrounds the ovum of animals. The egg coat provides structural support and can play an essential role in oogenesis, fertilization and early development. Also known as: structural constituent of vitelline envelope, structural constituent of zona pellucida Relationships: is a type of extracellular matrix structural constituent [GO:0005201]; occurs in GO:0035805